{
  "term_id": "UNKNOWN:0002",
  "gene_name": "MKRN2 opposite strand protein",
  "gene": "UniProtKB:H3BPM6",
  "gene_symbol": "MKRN2OS",
  "term_label": "Unknown biological process"
}